{
  "gene": "UniProtKB:P36406",
  "gene_name": "E3 ubiquitin-protein ligase TRIM23",
  "gene_symbol": "TRIM23",
  "term_id": "GO:0005886",
  "term_label": "plasma membrane"
}